{
  "term_id": "UNKNOWN:0002",
  "gene_name": "Inactive Ufm1-specific protease 1",
  "gene": "UniProtKB:Q6NVU6",
  "gene_symbol": "UFSP1",
  "term_label": "Unknown biological process"
}